quinate dehydrogenase (quinone) activity [GO:0047519] (MF) Also known as: quinate:quinone 3-oxidoreductase activity, NAD(P)-independent quinate dehydrogenase activity, quinate:pyrroloquinoline-quinone 5-oxidoreductase activity Sources: RHEA:23672 Definition: Catalysis of the reaction: (-)-quinate + pyrroloquinoline-quinone = (-)-3-dehydroquinate + pyrroloquinoline-quinol. Relationships: is a type of oxidoreductase activity, acting on the CH-OH group of donors, quinone or similar compound as acceptor [GO:0016901]